{
  "gene": "UniProtKB:O43709",
  "term_id": "GO:0070476",
  "term_label": "rRNA (guanine-N7)-methylation",
  "gene_symbol": "BUD23",
  "gene_name": "Probable 18S rRNA (guanine-N(7))-methyltransferase"
}